positive regulation of cell-substrate adhesion [GO:0010811] (biological process) Definition: Any process that increases the frequency, rate or extent of cell-substrate adhesion. Cell-substrate adhesion is the attachment of a cell to the underlying substrate via adhesion molecules. Relationships: is a type of GO:0010810; is a type of GO:0045785; positively regulates GO:0031589 Sources: GOC:dph, GOC:pf, GOC:tb Subtypes: GO:0001954, GO:1900026, positive regulation of cell adhesion involved in single-species biofilm formation [GO:1900189], positive regulation of substrate-dependent cell migration, cell attachment to substrate [GO:1904237]